{
  "gene_name": "Protein ATP6V1FNB",
  "term_id": "UNKNOWN:0003",
  "gene_symbol": "ATP6V1FNB",
  "gene": "UniProtKB:A0A1B0GUX0",
  "term_label": "Unknown cellular component"
}